corpus callosum morphogenesis [GO:0021540] (biological process) Sources: GOC:cls, GOC:dgh, GOC:dph, GOC:jid, GO_REF:0000021 Relationships: is a type of central nervous system projection neuron axonogenesis [GO:0021952]; is part of GO:0022038 Definition: The process in which the anatomical structures of the corpus callosum are generated and organized. The corpus callosum is a thick bundle of nerve fibers comprising a commissural plate connecting the two cerebral hemispheres. It consists of contralateral axon projections that provides communications between the right and left cerebral hemispheres.